{
  "gene": "UniProtKB:Q8IUB3",
  "gene_name": "Protein WFDC10B",
  "term_label": "serine-type endopeptidase inhibitor activity",
  "gene_symbol": "WFDC10B",
  "term_id": "GO:0004867"
}